{
  "term_id": "GO:0051726",
  "term_label": "regulation of cell cycle",
  "gene_name": "Protein lin-9 homolog",
  "gene": "UniProtKB:Q5TKA1",
  "gene_symbol": "LIN9"
}